{
  "term_label": "regulation of DNA-templated transcription",
  "gene": "UniProtKB:P51587",
  "gene_symbol": "BRCA2",
  "gene_name": "Breast cancer type 2 susceptibility protein",
  "term_id": "GO:0006355"
}